Dom34-Hbs1 complex [GO:1990533] (cellular component) Definition: A protein complex consisting of one subunit known as Dom34 or Pelota that has similarity to translation termination factor eRF1, and another subunit, Hbs1, that is a GTPase with similarity to translation termination factor eRF3. The Dom34-Hbs1 complex has a role in cotranslational mRNA quality control by promoting ribosomal subunit dissociation and peptidyl-tRNA release when translation is stalled, facilitating no-go decay and nonstop decay. References: PMID:20890290, PMID:21102444, PMID:21448132, PMID:22503425 Sources: GOC:mcc Relationships: is a type of protein-containing complex [GO:0032991] Also known as: Dom34:Hbs1 complex